{
  "gene_symbol": "COQ9",
  "gene_name": "Ubiquinone biosynthesis protein COQ9, mitochondrial",
  "term_label": "ubiquinone biosynthetic process",
  "gene": "UniProtKB:O75208",
  "term_id": "GO:0006744"
}